{
  "gene_name": "Histone H2B type F-S",
  "term_id": "GO:0003677",
  "gene_symbol": "H2BC12L",
  "term_label": "DNA binding",
  "gene": "UniProtKB:P57053"
}